{
  "gene_symbol": "RAD23B",
  "gene": "UniProtKB:P54727",
  "term_label": "ubiquitin binding",
  "gene_name": "UV excision repair protein RAD23 homolog B",
  "term_id": "GO:0043130"
}